{
  "gene": "UniProtKB:Q14508",
  "term_id": "GO:0019731",
  "gene_symbol": "WFDC2",
  "gene_name": "WAP four-disulfide core domain protein 2",
  "term_label": "antibacterial humoral response"
}